negative regulation of mesenchymal cell apoptotic process involved in mesonephric nephron morphogenesis [GO:0061296] (biological process) Sources: GOC:mtg_apoptosis, GOC:mtg_kidney_jan10 Also known as: negative regulation of mesenchymal stem cell apoptotic process involved in mesonephric nephron morphogenesis, negative regulation of mesenchymal stem cell apoptosis involved in mesonephric nephron morphogenesis Relationships: is a type of GO:0061218; is a type of regulation of mesenchymal cell apoptotic process involved in mesonephric nephron morphogenesis [GO:0061295]; is a type of GO:0072040; RO_0002212 mesenchymal stem cell maintenance involved in mesonephric nephron morphogenesis [GO:0061235]; negatively regulates GO:1901146 Definition: Any process that reduces the occurrence or rate of mesenchymal stem cell death by apoptotic process that contributes to the shaping of the nephron in the mesonephros.